{
  "term_id": "GO:0051500",
  "gene": "UniProtKB:Q8TEA8",
  "term_label": "D-tyrosyl-tRNA(Tyr) deacylase activity",
  "gene_symbol": "DTD1",
  "gene_name": "D-aminoacyl-tRNA deacylase 1"
}